{
  "gene_symbol": "CFAP20",
  "term_id": "GO:0060271",
  "gene": "UniProtKB:Q9Y6A4",
  "term_label": "cilium assembly",
  "gene_name": "Cilia- and flagella-associated protein 20"
}